clearance of cells from fusion plate by apoptotic process [GO:0060885] (biological process) Sources: GOC:dph, GOC:mtg_apoptosis, GOC:sdb_2009, GOC:tb Also known as: clearance of cells from fusion plate by apoptosis Definition: Any apoptotic process that contributes to the shaping of the semicircular canal by removing cells in the fusion plate, forming the loops of the canals. Relationships: is a type of apoptotic process involved in morphogenesis [GO:0060561]; is a type of GO:0060884